{
  "gene_symbol": "ADM2",
  "term_label": "adrenomedullin receptor signaling pathway",
  "gene": "UniProtKB:Q7Z4H4",
  "term_id": "GO:1990410",
  "gene_name": "Protein ADM2"
}